{
  "gene_name": "Interferon-induced protein with tetratricopeptide repeats 1B",
  "gene_symbol": "IFIT1B",
  "term_id": "GO:0003723",
  "term_label": "RNA binding",
  "gene": "UniProtKB:Q5T764"
}